nerve development [GO:0021675] (BP) Sources: GOC:cls, GOC:dgh, GOC:dph, GOC:jid, GO_REF:0000021 Relationships: is a type of GO:0048856; is part of GO:0007399 Subtypes: cranial nerve development [GO:0021545] Definition: The process whose specific outcome is the progression of a nerve over time, from its formation to the mature structure.